{
  "term_label": "phytanoyl-CoA dioxygenase activity",
  "gene_symbol": "PHYH",
  "gene_name": "Phytanoyl-CoA dioxygenase, peroxisomal",
  "gene": "UniProtKB:O14832",
  "term_id": "GO:0048244"
}